{
  "gene_symbol": "NMNAT3",
  "gene_name": "Nicotinamide_nicotinic acid mononucleotide adenylyltransferase 3",
  "term_label": "nicotinate-nucleotide adenylyltransferase activity",
  "gene": "UniProtKB:Q96T66",
  "term_id": "GO:0004515"
}